{
  "gene_name": "Zinc finger protein 681",
  "term_label": "RNA polymerase II cis-regulatory region sequence-specific DNA binding",
  "gene": "UniProtKB:Q96N22",
  "gene_symbol": "ZNF681",
  "term_id": "GO:0000978"
}